{
  "term_id": "GO:0031122",
  "gene_symbol": "TUBGCP6",
  "gene_name": "Gamma-tubulin complex component 6",
  "gene": "UniProtKB:Q96RT7",
  "term_label": "cytoplasmic microtubule organization"
}